{
  "gene_name": "Basic helix-loop-helix ARNT-like protein 1",
  "term_id": "GO:0006357",
  "gene": "UniProtKB:O00327",
  "term_label": "regulation of transcription by RNA polymerase II",
  "gene_symbol": "BMAL1"
}